{
  "term_id": "UNKNOWN:0002",
  "gene": "UniProtKB:Q9BW91",
  "gene_symbol": "NUDT9",
  "term_label": "Unknown biological process",
  "gene_name": "ADP-ribose pyrophosphatase, mitochondrial"
}